{
  "gene": "UniProtKB:Q6PI25",
  "term_label": "synapse",
  "term_id": "GO:0045202",
  "gene_name": "Protein cornichon homolog 2",
  "gene_symbol": "CNIH2"
}